calcium:proton antiporter activity [GO:0015369] (molecular function) Sources: RHEA:71799, TC:2.A.19.2.- Definition: Enables the transfer of a solute or solutes from one side of a membrane to the other according to the reaction: Ca2+(in) + H+(out) = Ca2+(out) + H+(in). Also known as: calcium:hydrogen antiporter activity Relationships: is a type of calcium:monoatomic cation antiporter activity [GO:0015368]; is a type of metal cation:proton antiporter activity [GO:0051139]